{
  "term_label": "endosomal transport",
  "gene_name": "Neuronal vesicle trafficking-associated protein 1",
  "gene_symbol": "NSG1",
  "term_id": "GO:0016197",
  "gene": "UniProtKB:P42857"
}